{
  "term_id": "GO:0090263",
  "gene_symbol": "PPM1A",
  "term_label": "positive regulation of canonical Wnt signaling pathway",
  "gene": "UniProtKB:P35813",
  "gene_name": "Protein phosphatase 1A"
}